negative regulation of intrinsic apoptotic signaling pathway in response to DNA damage by p53 class mediator [GO:1902166] (biological process) Definition: Any process that stops, prevents or reduces the frequency, rate or extent of intrinsic apoptotic signaling pathway in response to DNA damage by p53 class mediator. Relationships: is a type of GO:1902165; is a type of negative regulation of intrinsic apoptotic signaling pathway in response to DNA damage [GO:1902230]; is_a negative regulation of intrinsic apoptotic signaling pathway by p53 class mediator [GO:1902254]; negatively regulates intrinsic apoptotic signaling pathway in response to DNA damage by p53 class mediator [GO:0042771] References: PMID:17719541 Sources: GOC:TermGenie Also known as: down regulation of intrinsic apoptotic signaling pathway in response to DNA damage by p53 class mediator, down-regulation of intrinsic apoptotic signaling pathway in response to DNA damage by p53 class mediator, downregulation of intrinsic apoptotic signaling pathway in response to DNA damage by p53 class mediator, inhibition of intrinsic apoptotic signaling pathway in response to DNA damage by p53 class mediator, down regulation of DNA damage response, signal transduction by p53 class mediator resulting in induction of apoptosis, down-regulation of DNA damage response, signal transduction by p53 class mediator resulting in induction of apoptosis, downregulation of DNA damage response, signal transduction by p53 class mediator resulting in induction of apoptosis, inhibition of DNA damage response, signal transduction by p53 class mediator resulting in induction of apoptosis, negative regulation of DNA damage response, signal transduction by p53 class mediator resulting in induction of apoptosis